four-way junction helicase activity [GO:0009378] (molecular function) Also known as: ATP-dependent four-way junction DNA helicase activity, ATP-dependent four-way junction helicase activity, ATP-dependent Holliday junction helicase activity, Holliday junction helicase activity Relationships: is a type of DNA helicase activity [GO:0003678] References: PMID:22723423, PMID:9442895 Sources: GOC:al Definition: Unwinding a DNA helix of DNA containing four-way junctions, including Holliday junctions, driven by ATP hydrolysis.